succinate-CoA ligase (ADP-forming) activity [GO:0004775] (molecular function) References: PMID:9874242 Sources: RHEA:17661 Relationships: is a type of succinate-CoA ligase activity [GO:0004774] Definition: Catalysis of the reaction: ATP + succinate + CoA = ADP + succinyl-CoA + phosphate. Also known as: succinic thiokinase, succinyl coenzyme A synthetase, succinate thiokinase activity, succinyl coenzyme A synthetase (adenosine diphosphate-forming) activity, succinyl-CoA synthetase (ADP-forming) activity, succinyl-CoA synthetase activity